fructose transmembrane transporter activity [GO:0005353] (molecular function) Subtypes: GO:0015284, GO:0022877, fructose:proton symporter activity [GO:0055054], high-affinity fructose transmembrane transporter activity [GO:0061486], GO:0140930 Definition: Enables the transfer of fructose from one side of a membrane to the other. Fructose exists in a open chain form or as a ring compound. D-fructose is the sweetest of the sugars and is found free in a large number of fruits and honey. Relationships: is a type of GO:0015149; is part of fructose transmembrane transport [GO:0015755] Sources: GOC:ai, GOC:mtg_transport, ISBN:0815340729 Also known as: fructose permease activity, fructose porter activity